{
  "gene_symbol": "KLHL22",
  "gene_name": "Kelch-like protein 22",
  "term_label": "mitotic spindle",
  "gene": "UniProtKB:Q53GT1",
  "term_id": "GO:0072686"
}